{
  "gene_symbol": "C1orf174",
  "gene": "UniProtKB:Q8IYL3",
  "term_label": "Unknown molecular function",
  "gene_name": "UPF0688 protein C1orf174",
  "term_id": "UNKNOWN:0001"
}